{
  "gene_symbol": "GPER1",
  "term_id": "GO:0005794",
  "gene": "UniProtKB:Q99527",
  "gene_name": "G-protein coupled estrogen receptor 1",
  "term_label": "Golgi apparatus"
}